{
  "term_id": "GO:0000981",
  "gene": "UniProtKB:O43812",
  "gene_name": "Double homeobox protein 1",
  "term_label": "DNA-binding transcription factor activity, RNA polymerase II-specific",
  "gene_symbol": "DUX1"
}